{
  "gene_symbol": "EMX1",
  "gene_name": "Homeobox protein EMX1",
  "gene": "UniProtKB:Q04741",
  "term_label": "nucleus",
  "term_id": "GO:0005634"
}